{
  "gene_symbol": "ELMO1",
  "gene": "UniProtKB:Q92556",
  "term_id": "GO:0032045",
  "term_label": "guanyl-nucleotide exchange factor complex",
  "gene_name": "Engulfment and cell motility protein 1"
}